regulation of sprouting angiogenesis [GO:1903670] (biological process) Definition: Any process that modulates the frequency, rate or extent of sprouting angiogenesis. References: PMID:16756958 Sources: GOC:TermGenie, GO_REF:0000058 Subtypes: GO:1903671, GO:1903672 Relationships: is a type of GO:0045765; regulates sprouting angiogenesis [GO:0002040]